{
  "gene_name": "KRAB-A domain-containing protein 2",
  "term_id": "UNKNOWN:0003",
  "gene": "UniProtKB:Q6ZNG9",
  "gene_symbol": "KRBA2",
  "term_label": "Unknown cellular component"
}